{
  "term_id": "GO:0005096",
  "term_label": "GTPase activator activity",
  "gene_symbol": "SEC23A",
  "gene": "UniProtKB:Q15436",
  "gene_name": "Protein transport protein Sec23A"
}